{
  "gene_symbol": "CDH24",
  "term_id": "GO:0034332",
  "gene_name": "Cadherin-24",
  "term_label": "adherens junction organization",
  "gene": "UniProtKB:Q86UP0"
}